{
  "term_label": "Unknown molecular function",
  "term_id": "UNKNOWN:0001",
  "gene_symbol": "BBS9",
  "gene": "UniProtKB:Q3SYG4",
  "gene_name": "Protein PTHB1"
}